{
  "gene": "UniProtKB:Q8NGC7",
  "term_id": "UNKNOWN:0002",
  "term_label": "Unknown biological process",
  "gene_symbol": "OR11H6",
  "gene_name": "Olfactory receptor 11H6"
}